{
  "term_id": "GO:0005829",
  "gene_symbol": "AMFR",
  "gene": "UniProtKB:Q9UKV5",
  "gene_name": "E3 ubiquitin-protein ligase AMFR",
  "term_label": "cytosol"
}